testosterone biosynthetic process [GO:0061370] (BP) Definition: The chemical reactions and pathways resulting in the formation of testosterone, an androgen having 17beta-hydroxy and 3-oxo groups, together with unsaturation at C-4 C-5. Sources: GOC:dph, GOC:yaf Relationships: is a type of steroid biosynthetic process [GO:0006694]; is_a ketone biosynthetic process [GO:0042181]; is a type of GO:0120255 Regulation: regulated by regulation of testosterone biosynthetic process [GO:2000224]; RO_0002212 by GO:2000225